{
  "term_label": "cytoplasm",
  "gene": "UniProtKB:Q9Y216",
  "gene_symbol": "MTMR7",
  "term_id": "GO:0005737",
  "gene_name": "Myotubularin-related protein 7"
}